{
  "term_id": "GO:0004888",
  "term_label": "transmembrane signaling receptor activity",
  "gene": "UniProtKB:A0A191URJ7",
  "gene_name": "KIR2DL protein",
  "gene_symbol": "KIR2DL1"
}